{
  "term_id": "UNKNOWN:0001",
  "gene_name": "Uncharacterized protein",
  "gene": "UniProtKB:A0A1B0GVB3",
  "term_label": "Unknown molecular function",
  "gene_symbol": "LOC102725191"
}